{
  "gene": "UniProtKB:Q9HBE5",
  "term_id": "GO:0004896",
  "gene_name": "Interleukin-21 receptor",
  "gene_symbol": "IL21R",
  "term_label": "cytokine receptor activity"
}